{
  "term_id": "UNKNOWN:0001",
  "gene_name": "Lipase maturation factor 1",
  "gene": "UniProtKB:Q96S06",
  "gene_symbol": "LMF1",
  "term_label": "Unknown molecular function"
}